{
  "gene_name": "Beta-defensin 125",
  "term_label": "killing of cells of another organism",
  "gene_symbol": "DEFB125",
  "gene": "UniProtKB:Q8N687",
  "term_id": "GO:0031640"
}